{
  "term_id": "GO:0005764",
  "gene_name": "Cathepsin D",
  "gene": "UniProtKB:P07339",
  "term_label": "lysosome",
  "gene_symbol": "CTSD"
}